{
  "term_label": "apical protein localization",
  "term_id": "GO:0045176",
  "gene_symbol": "INSC",
  "gene": "UniProtKB:Q1MX18",
  "gene_name": "Protein inscuteable homolog"
}